neurotransmitter receptor transport, postsynaptic endosome to lysosome [GO:0098943] (biological process) Sources: GOC:dos Relationships: is a type of GO:0006886; is a type of endosome to lysosome transport [GO:0008333]; is a type of protein localization to lysosome [GO:0061462]; is a type of GO:0072666; is a type of GO:0099637 Also known as: postsynaptic neurotransmitter receptor endosomal trafficking Definition: The directed movement of neurotransmitter receptor from the postsynaptic endosome in tranpsort vesicles to the lysosome for degradation.